{
  "term_id": "GO:0031430",
  "gene_symbol": "MYOM3",
  "term_label": "M band",
  "gene": "UniProtKB:Q5VTT5",
  "gene_name": "Myomesin-3"
}